{
  "gene_name": "Fascin-3",
  "gene": "UniProtKB:Q9NQT6",
  "term_label": "actin filament bundle assembly",
  "term_id": "GO:0051017",
  "gene_symbol": "FSCN3"
}